{
  "gene_name": "XK-related protein 8",
  "gene": "UniProtKB:Q9H6D3",
  "term_id": "GO:0043652",
  "term_label": "engulfment of apoptotic cell",
  "gene_symbol": "XKR8"
}